{
  "gene": "UniProtKB:P02647",
  "term_label": "low-density lipoprotein particle",
  "term_id": "GO:0034362",
  "gene_symbol": "APOA1",
  "gene_name": "Apolipoprotein A-I"
}